{
  "term_label": "Unknown cellular component",
  "gene_name": "Putative C-mannosyltransferase DPY19L2P1",
  "gene": "UniProtKB:Q6NXN4",
  "gene_symbol": "DPY19L2P1",
  "term_id": "UNKNOWN:0003"
}